{
  "term_label": "DNA topoisomerase type I (single strand cut, ATP-independent) activity",
  "gene_name": "DNA topoisomerase 3-alpha",
  "term_id": "GO:0003917",
  "gene": "UniProtKB:Q13472",
  "gene_symbol": "TOP3A"
}